negative regulation of cyclic-nucleotide phosphodiesterase activity [GO:0051344] (biological process) Definition: Any process that stops or reduces the rate of cyclic nucleotide phosphodiesterase activity, the catalysis of the reaction: nucleotide 3',5'-cyclic phosphate + H2O = nucleotide 5'-phosphate. Sources: GOC:ai, GOC:tb Also known as: 3',5' cyclic nucleotide phosphodiesterase inhibitor, down regulation of cyclic nucleotide phosphodiesterase activity, down-regulation of cyclic nucleotide phosphodiesterase activity, downregulation of cyclic nucleotide phosphodiesterase activity, negative regulation of 3',5' cyclic nucleotide phosphodiesterase activity, negative regulation of cyclic nucleotide phosphodiesterase activity, 3',5'-cyclic-AMP phosphodiesterase inhibitor, cAMP phosphodiesterase inhibitor, inhibition of cyclic nucleotide phosphodiesterase activity, negative regulation of 3',5'-cyclic-AMP phosphodiesterase activity, negative regulation of cAMP phosphodiesterase activity, negative regulation of cGMP phosphodiesterase activity, phosphodiesterase inhibitor Relationships: is_a negative regulation of hydrolase activity [GO:0051346]; negatively regulates GO:0004112